cellular response to leukemia inhibitory factor [GO:1990830] (biological process) References: PMID:12801913 Definition: Any process that results in a change in state or activity of a cell (in terms of movement, secretion, enzyme production, gene expression, etc.) as a result of a leukemia inhibitory factor stimulus. Also known as: cellular response to CDF, cellular response to cholinergic differentiation factor Relationships: is a type of cellular response to cytokine stimulus [GO:0071345]; is a type of response to leukemia inhibitory factor [GO:1990823]